{
  "term_id": "GO:0000932",
  "term_label": "P-body",
  "gene_symbol": "CNOT9",
  "gene": "UniProtKB:Q92600",
  "gene_name": "CCR4-NOT transcription complex subunit 9"
}